anthranilate 1,2-dioxygenase (deaminating, decarboxylating) activity [GO:0018618] (molecular function) Also known as: anthranilate hydroxylase activity, anthranilic acid hydroxylase activity, anthranilic hydroxylase activity, anthranilate dioxygenase activity, anthranilate dioxygenase reductase, AntA, AntB, AntC, anthranilate 1,2-dioxygenase, anthranilate,NAD(P)H:oxygen oxidoreductase (1,2-hydroxylating, deaminating, decarboxylating) Sources: EC:1.14.12.1 Definition: Catalysis of the reaction: anthranilate + NADPH + H+ + O2 = catechol + CO2 + NADP+ + NH3. Relationships: is a type of oxidoreductase activity, acting on paired donors, with incorporation or reduction of molecular oxygen, NAD(P)H as one donor, and incorporation of two atoms of oxygen into one donor [GO:0016708]